{
  "gene_symbol": "PRSS12",
  "gene": "UniProtKB:P56730",
  "term_id": "GO:0098978",
  "term_label": "glutamatergic synapse",
  "gene_name": "Neurotrypsin"
}